{
  "gene_name": "T-cell leukemia homeobox protein 2",
  "term_id": "GO:0005634",
  "gene_symbol": "TLX2",
  "term_label": "nucleus",
  "gene": "UniProtKB:O43763"
}